{
  "term_label": "tight junction assembly",
  "gene": "UniProtKB:O00501",
  "term_id": "GO:0120192",
  "gene_name": "Claudin-5",
  "gene_symbol": "CLDN5"
}